collagen type XXIV trimer [GO:1990323] (cellular component) Definition: A collagen homotrimer of alpha1(XXIV) chains; type XXIV collagen triple helices may participate in regulating type I collagen fibrillogenesis at specific anatomical locations during fetal development. References: PMID:17876790 Sources: GOC:bhm Relationships: is a type of fibrillar collagen trimer [GO:0005583]